{
  "gene": "UniProtKB:Q96PS6",
  "gene_symbol": "GAFA1",
  "term_label": "Unknown cellular component",
  "term_id": "UNKNOWN:0003",
  "gene_name": "Putative uncharacterized protein GAFA-1"
}